{
  "gene_symbol": "RNF149",
  "term_id": "GO:0061630",
  "term_label": "ubiquitin protein ligase activity",
  "gene": "UniProtKB:Q8NC42",
  "gene_name": "E3 ubiquitin-protein ligase RNF149"
}